aromatic amino acid metabolic process [GO:0009072] (biological process) Sources: GOC:go_curators Subtypes: L-histidine metabolic process [GO:0006547], L-phenylalanine metabolic process [GO:0006558], L-tryptophan metabolic process [GO:0006568], tyrosine metabolic process [GO:0006570], serotonin biosynthetic process from tryptophan [GO:0006587], aromatic amino acid family biosynthetic process [GO:0009073], aromatic amino acid family catabolic process [GO:0009074], GO:0019356, anthranilate metabolic process [GO:0043420], GO:0046482, L-dopa metabolic process [GO:1903184] Definition: The chemical reactions and pathways involving aromatic amino acid family, amino acids with aromatic ring (phenylalanine, tyrosine, tryptophan). Also known as: aromatic amino acid family metabolic process, aromatic amino acid family metabolism Relationships: is a type of amino acid metabolic process [GO:0006520]; is a type of carboxylic acid metabolic process [GO:0019752]